{
  "gene": "UniProtKB:P24522",
  "term_label": "regulation of cell cycle",
  "gene_symbol": "GADD45A",
  "gene_name": "Growth arrest and DNA damage-inducible protein GADD45 alpha",
  "term_id": "GO:0051726"
}